negative regulation of myeloid leukocyte differentiation [GO:0002762] (biological process) Relationships: is a type of regulation of myeloid leukocyte differentiation [GO:0002761]; is a type of GO:0045638; is a type of GO:1902106; negatively regulates myeloid leukocyte differentiation [GO:0002573] Also known as: down regulation of myeloid leukocyte differentiation, down-regulation of myeloid leukocyte differentiation, downregulation of myeloid leukocyte differentiation, inhibition of myeloid leukocyte differentiation Subtypes: negative regulation of granulocyte differentiation [GO:0030853], GO:0045650, GO:0045656, negative regulation of osteoclast differentiation [GO:0045671], negative regulation of mast cell differentiation [GO:0060377] Definition: Any process that stops, prevents, or reduces the frequency, rate, or extent of myeloid leukocyte differentiation. Sources: GOC:add